{
  "gene_symbol": "RNASE10",
  "gene": "UniProtKB:Q5GAN6",
  "term_label": "Unknown molecular function",
  "gene_name": "Inactive ribonuclease-like protein 10",
  "term_id": "UNKNOWN:0001"
}